external encapsulating structure [GO:0030312] (cellular component) Subtypes: cell wall [GO:0005618], glycocalyx [GO:0030112], S-layer [GO:0030115], GO:0031012, egg chorion [GO:0042600], pollen wall [GO:0043667], GO:0140139, collagenous component of basement membrane [GO:0140143], non-collagenous component of basement membrane [GO:0140144], gel phase of basement membrane [GO:0140148], GO:0140149, GO:0140150, solid phase of interstitial matrix [GO:0140151], collagenous component of interstitial matrix [GO:0140152] Relationships: is a type of cellular anatomical structure [GO:0110165]; is part of GO:0071944 Sources: GOC:go_curators Note: The outer membrane (of gram negative bacteria) or cell wall (of yeast or Gram positive bacteria) are defined as parts of this structure, see 'external encapsulating structure part'. Definition: A structure that lies outside the plasma membrane and surrounds the entire cell or cells. This does not include the periplasmic space.